{
  "term_id": "UNKNOWN:0001",
  "gene_symbol": "TRAJ45",
  "term_label": "Unknown molecular function",
  "gene": "UniProtKB:A0A075B6X0",
  "gene_name": "T cell receptor alpha joining 45 (Fragment)"
}